{
  "gene_name": "Potassium-transporting ATPase alpha chain 1",
  "gene_symbol": "ATP4A",
  "term_label": "P-type potassium:proton transporter activity",
  "gene": "UniProtKB:P20648",
  "term_id": "GO:0008900"
}